{
  "gene": "UniProtKB:Q96QU8",
  "gene_name": "Exportin-6",
  "term_id": "UNKNOWN:0003",
  "gene_symbol": "XPO6",
  "term_label": "Unknown cellular component"
}